{
  "gene_symbol": "LILRA1",
  "gene_name": "Leukocyte immunoglobulin-like receptor subfamily A member 1",
  "term_label": "plasma membrane",
  "gene": "UniProtKB:O75019",
  "term_id": "GO:0005886"
}